{
  "term_label": "Unknown cellular component",
  "gene_name": "E3 ubiquitin-protein ligase RNF5",
  "gene_symbol": "RNF5",
  "term_id": "UNKNOWN:0003",
  "gene": "UniProtKB:Q99942"
}